{
  "term_id": "GO:0005634",
  "gene": "UniProtKB:Q86U44",
  "gene_name": "N6-adenosine-methyltransferase catalytic subunit",
  "gene_symbol": "METTL3",
  "term_label": "nucleus"
}